{
  "term_id": "GO:0005525",
  "term_label": "GTP binding",
  "gene": "UniProtKB:P63000",
  "gene_name": "Ras-related C3 botulinum toxin substrate 1",
  "gene_symbol": "RAC1"
}